{
  "gene": "UniProtKB:Q15223",
  "term_id": "GO:0007157",
  "gene_symbol": "NECTIN1",
  "term_label": "heterophilic cell-cell adhesion",
  "gene_name": "Nectin-1"
}